{
  "gene_symbol": "CATSPER3",
  "term_id": "GO:0030317",
  "gene_name": "Cation channel sperm-associated protein 3",
  "gene": "UniProtKB:Q86XQ3",
  "term_label": "flagellated sperm motility"
}